{
  "gene_symbol": "ZSCAN1",
  "gene": "UniProtKB:Q8NBB4",
  "term_id": "GO:0000978",
  "gene_name": "Zinc finger and SCAN domain-containing protein 1",
  "term_label": "RNA polymerase II cis-regulatory region sequence-specific DNA binding"
}